cytosine:proton symporter activity [GO:0015504] (molecular function) Sources: TC:2.A.39.1.1 Also known as: cytosine:hydrogen ion symporter activity, cytosine permease activity Definition: Enables the transfer of a solute or solutes from one side of a membrane to the other according to the reaction: cytosine(out) + H+(out) = cytosine(in) + H+(in). Relationships: is_a cytosine transmembrane transporter activity [GO:0015209]; is a type of solute:proton symporter activity [GO:0015295]; is a type of nucleobase:monoatomic cation symporter activity [GO:0015391]